propionate catabolic process [GO:0019543] (biological process) Definition: The chemical reactions and pathways resulting in the breakdown of propionate, the anion derived from propionic acid. Sources: GOC:go_curators Also known as: propionate breakdown, propionate catabolism, propionate degradation Relationships: is a type of propionate metabolic process [GO:0019541]; is a type of GO:0019626 Subtypes: propionate catabolic process, 2-methylcitrate cycle [GO:0019629]